{
  "gene_symbol": "SLC52A2",
  "gene_name": "Solute carrier family 52, riboflavin transporter, member 2",
  "gene": "UniProtKB:Q9HAB3",
  "term_id": "GO:0005886",
  "term_label": "plasma membrane"
}